{
  "gene_symbol": "KCNK13",
  "gene_name": "Potassium channel subfamily K member 13",
  "term_label": "outward rectifier potassium channel activity",
  "term_id": "GO:0015271",
  "gene": "UniProtKB:Q9HB14"
}